{
  "gene_symbol": "LSAMP",
  "term_id": "GO:0051963",
  "gene": "UniProtKB:Q13449",
  "term_label": "regulation of synapse assembly",
  "gene_name": "Limbic system-associated membrane protein"
}